positive regulation of CD4-positive, alpha-beta T cell activation [GO:2000516] (biological process) Sources: GOC:obol Relationships: is a type of GO:0046635; is a type of regulation of CD4-positive, alpha-beta T cell activation [GO:2000514]; positively regulates CD4-positive, alpha-beta T cell activation [GO:0035710] Subtypes: GO:0035783, positive regulation of CD4-positive, alpha-beta T cell differentiation [GO:0043372], GO:1900281, GO:2000519, positive regulation of CD4-positive, alpha-beta T cell proliferation [GO:2000563], positive regulation of T-helper 2 cell activation [GO:2000570] Definition: Any process that activates or increases the frequency, rate or extent of CD4-positive, alpha-beta T cell activation.